olfactory bulb interneuron fate commitment [GO:0021890] (biological process) References: PMID:12626695 Sources: GOC:cls, GOC:dgh, GOC:dph, GOC:jid, GO_REF:0000021 Relationships: is a type of neuron fate commitment [GO:0048663]; is part of olfactory bulb interneuron differentiation [GO:0021889] Definition: The process in which the developmental fate of a neuroblast becomes restricted such that it will develop into an interneuron residing in the olfactory bulb.